{
  "gene": "UniProtKB:Q16637",
  "term_id": "GO:0007409",
  "term_label": "axonogenesis",
  "gene_symbol": "SMN2",
  "gene_name": "Survival motor neuron protein"
}